positive regulation of apoptotic cell clearance [GO:2000427] (biological process) Definition: Any process that activates or increases the frequency, rate or extent of apoptotic cell clearance. Sources: GOC:obol Subtypes: GO:1901076 Relationships: is a type of positive regulation of phagocytosis [GO:0050766]; is a type of GO:2000425; positively regulates apoptotic cell clearance [GO:0043277] Also known as: positive regulation of apoptotic cell removal, positive regulation of efferocytosis, positive regulation of programmed cell clearance